regulation of type B pancreatic cell proliferation [GO:0061469] (biological process) Relationships: is a type of GO:0050678; regulates type B pancreatic cell proliferation [GO:0044342] Definition: Any process that modulates the frequency, rate or extent of type B pancreatic cell proliferation. Sources: GOC:dph Subtypes: GO:1904691, positive regulation of type B pancreatic cell proliferation [GO:1904692]